symbiont entry into host cell via permeabilization of inner membrane [GO:0099008] (biological process) References: PMID:15795287, PMID:20427561 Relationships: is_a symbiont entry into host cell via permeabilization of host membrane [GO:0140267] Also known as: viral entry via permeabilization of inner membrane Definition: The entry of a symbiont into the cytoplasm of a host cell, following fusion with the outer membrane, via permeabilization of the plasma (inner) membrane. This process mediates the entry of some non-enveloped viruses into prokaryotic cells. In the case of some double stranded RNA viruses of prokaryotes this occurs via interaction of a membrane-interacting component of the capsid, leading to depolarization and permeabilization of the plasma membrane.